{
  "term_id": "GO:0060005",
  "gene_name": "Transmembrane channel-like protein 1",
  "gene": "UniProtKB:Q8TDI8",
  "term_label": "vestibular reflex",
  "gene_symbol": "TMC1"
}